{
  "term_id": "GO:0010468",
  "term_label": "regulation of gene expression",
  "gene_symbol": "TRIM49D1",
  "gene_name": "Tripartite motif-containing protein 49D",
  "gene": "UniProtKB:C9J1S8"
}